{
  "gene_symbol": "NAT14",
  "term_label": "Unknown biological process",
  "gene_name": "Probable N-acetyltransferase 14",
  "term_id": "UNKNOWN:0002",
  "gene": "UniProtKB:Q8WUY8"
}